{
  "term_label": "Unknown cellular component",
  "term_id": "UNKNOWN:0003",
  "gene_name": "Uncharacterized protein CSNK1G2-AS1",
  "gene_symbol": "CSNK1G2-AS1",
  "gene": "UniProtKB:Q8NCQ2"
}